regulation of methane biosynthetic process from 3-(methylthio)propionic acid [GO:1900333] (biological process) Definition: Any process that modulates the frequency, rate or extent of methane biosynthetic process from 3-(methylthio)propionic acid. Subtypes: negative regulation of methane biosynthetic process from 3-(methylthio)propionic acid [GO:1900334], positive regulation of methane biosynthetic process from 3-(methylthio)propionic acid [GO:1900335] Sources: GOC:TermGenie, GOC:mengo_curators Relationships: is a type of regulation of fatty acid metabolic process [GO:0019217]; is a type of regulation of sulfur metabolic process [GO:0042762]; is a type of regulation of cellular respiration [GO:0043457]; is a type of regulation of alkane biosynthetic process [GO:1901577]; regulates methane biosynthetic process from 3-(methylthio)propionic acid [GO:2001132]